{
  "term_label": "RNA polymerase II cis-regulatory region sequence-specific DNA binding",
  "gene_symbol": "TCF3",
  "gene_name": "Transcription factor E2-alpha",
  "term_id": "GO:0000978",
  "gene": "UniProtKB:P15923"
}